{
  "gene_symbol": "RAD51C",
  "gene_name": "DNA repair protein RAD51 homolog 3",
  "gene": "UniProtKB:O43502",
  "term_id": "GO:0005657",
  "term_label": "replication fork"
}